{
  "gene": "UniProtKB:Q9H237",
  "term_label": "membrane",
  "term_id": "GO:0016020",
  "gene_symbol": "PORCN",
  "gene_name": "Protein-serine O-palmitoleoyltransferase porcupine"
}